{
  "gene_name": "Cyclin-J",
  "term_label": "nucleus",
  "gene_symbol": "CCNJ",
  "gene": "UniProtKB:Q5T5M9",
  "term_id": "GO:0005634"
}